{
  "gene_symbol": "EPN2",
  "term_id": "GO:0006897",
  "term_label": "endocytosis",
  "gene": "UniProtKB:O95208",
  "gene_name": "Epsin-2"
}